{
  "gene": "UniProtKB:Q9UIK4",
  "gene_symbol": "DAPK2",
  "term_id": "GO:0035556",
  "term_label": "intracellular signal transduction",
  "gene_name": "Death-associated protein kinase 2"
}